negative regulation of Golgi lumen acidification [GO:1905527] (biological process) Also known as: down regulation of Golgi lumen acidification, down-regulation of Golgi lumen acidification, downregulation of Golgi lumen acidification, inhibition of Golgi lumen acidification References: PMID:23447592 Sources: GOC:TermGenie, GOC:dph, GO_REF:0000058 Relationships: is a type of negative regulation of cellular pH reduction [GO:0032848]; is a type of regulation of Golgi lumen acidification [GO:1905526]; negatively regulates Golgi lumen acidification [GO:0061795] Definition: Any process that stops, prevents or reduces the frequency, rate or extent of Golgi lumen acidification.